{
  "gene_symbol": "GGA1",
  "gene": "UniProtKB:Q9UJY5",
  "gene_name": "ADP-ribosylation factor-binding protein GGA1",
  "term_id": "GO:0005802",
  "term_label": "trans-Golgi network"
}